{
  "gene": "UniProtKB:Q13616",
  "gene_symbol": "CUL1",
  "gene_name": "Cullin-1",
  "term_id": "GO:0160072",
  "term_label": "ubiquitin ligase complex scaffold activity"
}